{
  "term_label": "extracellular space",
  "gene_name": "Complement component receptor 1-like protein",
  "term_id": "GO:0005615",
  "gene_symbol": "CR1L",
  "gene": "UniProtKB:Q2VPA4"
}